radial pattern formation [GO:0009956] (biological process) Subtypes: GO:0060771, root radial pattern formation [GO:0090057] Relationships: is a type of GO:0003002 Regulation: regulated by regulation of radial pattern formation [GO:0090213] Also known as: radial pattern specification Sources: GOC:dph, GOC:go_curators, GOC:isa_complete Definition: The regionalization process that results in defined areas around a point in which specific types of cell differentiation will occur.